{
  "gene_name": "Coiled-coil domain-containing protein 92",
  "term_id": "GO:0005814",
  "term_label": "centriole",
  "gene": "UniProtKB:Q53HC0",
  "gene_symbol": "CCDC92"
}